{
  "gene": "UniProtKB:O95833",
  "gene_name": "Chloride intracellular channel protein 3",
  "gene_symbol": "CLIC3",
  "term_id": "GO:0005254",
  "term_label": "chloride channel activity"
}